{
  "gene_name": "Protein O-glucosyltransferase 3",
  "term_id": "UNKNOWN:0002",
  "term_label": "Unknown biological process",
  "gene_symbol": "POGLUT3",
  "gene": "UniProtKB:Q7Z4H8"
}